negative regulation of TRAIL-activated apoptotic signaling pathway [GO:1903122] (biological process) Relationships: is a type of negative regulation of extrinsic apoptotic signaling pathway via death domain receptors [GO:1902042]; is a type of regulation of TRAIL-activated apoptotic signaling pathway [GO:1903121]; negatively regulates TRAIL-activated apoptotic signaling pathway [GO:0036462] Definition: Any process that stops, prevents or reduces the frequency, rate or extent of TRAIL-activated apoptotic signaling pathway. Also known as: down regulation of TRAIL-activated apoptotic signaling pathway, down regulation of TRAIL-activated extrinsic apoptotic signaling pathway, down regulation of TRAIL-induced apoptotic signaling pathway, down regulation of tumor necrosis factor-related apoptosis-inducing ligand apoptotic signaling pathway, down-regulation of TRAIL-activated apoptotic signaling pathway, down-regulation of TRAIL-activated extrinsic apoptotic signaling pathway, down-regulation of TRAIL-induced apoptotic signaling pathway, down-regulation of tumor necrosis factor-related apoptosis-inducing ligand apoptotic signaling pathway, downregulation of TRAIL-activated apoptotic signaling pathway, downregulation of TRAIL-activated extrinsic apoptotic signaling pathway, downregulation of TRAIL-induced apoptotic signaling pathway, downregulation of tumor necrosis factor-related apoptosis-inducing ligand apoptotic signaling pathway, negative regulation of TRAIL-activated extrinsic apoptotic signaling pathway, negative regulation of TRAIL-induced apoptotic signaling pathway, negative regulation of tumor necrosis factor-related apoptosis-inducing ligand apoptotic signaling pathway, inhibition of TRAIL-activated apoptotic signaling pathway, inhibition of TRAIL-activated extrinsic apoptotic signaling pathway, inhibition of TRAIL-induced apoptotic signaling pathway, inhibition of tumor necrosis factor-related apoptosis-inducing ligand apoptotic signaling pathway References: PMID:21785459 Sources: GOC:PARL, GOC:TermGenie, GOC:bf, GO_REF:0000058